tRNA-specific ribonuclease activity [GO:0004549] (molecular function) Subtypes: tRNA-intron lyase activity [GO:0000213], ribonuclease P activity [GO:0004526], 3'-tRNA processing endoribonuclease activity [GO:0042781] Also known as: tRNA-specific RNase activity Definition: Catalysis of the hydrolysis of phosphodiester bonds in tRNA molecules. Relationships: is a type of RNA nuclease activity [GO:0004540]; is a type of catalytic activity, acting on a tRNA [GO:0140101] Sources: GOC:mah